{
  "term_label": "Unknown cellular component",
  "term_id": "UNKNOWN:0003",
  "gene_name": "Cone cGMP-specific 3',5'-cyclic phosphodiesterase subunit alpha'",
  "gene_symbol": "PDE6C",
  "gene": "UniProtKB:P51160"
}